{
  "term_id": "GO:0003924",
  "term_label": "GTPase activity",
  "gene_name": "Atlastin-2",
  "gene": "UniProtKB:Q8NHH9",
  "gene_symbol": "ATL2"
}